{
  "gene_symbol": "PRRT1B",
  "term_label": "Unknown biological process",
  "term_id": "UNKNOWN:0002",
  "gene_name": "Proline rich transmembrane protein 1B",
  "gene": "UniProtKB:A0A1B0GWB2"
}